positive regulation of intermediate filament polymerization [GO:0030841] (biological process) Definition: Any process that activates or increases the frequency, rate or extent of intermediate filament polymerization. Sources: GOC:mah Also known as: positive regulation of intermediate filament polymerization and/or depolymerization, up regulation of intermediate filament polymerization, up-regulation of intermediate filament polymerization, upregulation of intermediate filament polymerization, activation of intermediate filament polymerization, stimulation of intermediate filament polymerization Note: Note that this term was split from 'positive regulation of intermediate filament polymerization and/or depolymerization ; GO:0045826' (sibling term 'positive regulation of intermediate filament depolymerization ; GO:0030844'). Relationships: is a type of GO:0030839; is a type of positive regulation of protein polymerization [GO:0032273]; is a type of positive regulation of cytoskeleton organization [GO:0051495]; positively regulates intermediate filament polymerization [GO:0045107]